{
  "gene_name": "Nuclear pore complex-interacting protein family member B13",
  "term_id": "UNKNOWN:0003",
  "term_label": "Unknown cellular component",
  "gene": "UniProtKB:A6NJU9",
  "gene_symbol": "NPIPB13"
}